{
  "gene_symbol": "LINC03043",
  "term_label": "Unknown molecular function",
  "gene_name": "Uncharacterized protein encoded by LINC03043",
  "gene": "UniProtKB:A4D0Y5",
  "term_id": "UNKNOWN:0001"
}